{
  "term_id": "GO:0004875",
  "term_label": "complement receptor activity",
  "gene": "UniProtKB:P21462",
  "gene_symbol": "FPR1",
  "gene_name": "fMet-Leu-Phe receptor"
}